regulation of glucuronoxylan catabolic process [GO:2000915] (biological process) Relationships: is a type of regulation of xylan catabolic process [GO:2001000]; regulates glucuronoxylan catabolic process [GO:2000886] Definition: Any process that modulates the frequency, rate or extent of glucuronoxylan catabolic process. Also known as: regulation of glucuronoxylan catabolism Sources: GOC:mengo_curators Subtypes: negative regulation of glucuronoxylan catabolic process [GO:2000916], GO:2000917, regulation of glucuronoarabinoxylan catabolic process [GO:2000918]